{
  "gene_name": "Protein FAM171A1",
  "gene_symbol": "FAM171A1",
  "term_id": "GO:0005886",
  "gene": "UniProtKB:Q5VUB5",
  "term_label": "plasma membrane"
}